{
  "gene_symbol": "SECISBP2",
  "term_label": "mRNA 3'-UTR binding",
  "gene_name": "Selenocysteine insertion sequence-binding protein 2",
  "gene": "UniProtKB:Q96T21",
  "term_id": "GO:0003730"
}